{
  "gene_symbol": "FBXO11",
  "term_id": "UNKNOWN:0001",
  "gene": "UniProtKB:Q86XK2",
  "gene_name": "F-box only protein 11",
  "term_label": "Unknown molecular function"
}